negative regulation of cellulosome assembly [GO:1900504] (biological process) Definition: Any process that stops, prevents or reduces the frequency, rate or extent of cellulosome assembly. Sources: GOC:TermGenie, GOC:mengo_curators Relationships: is a type of GO:1900503; is a type of negative regulation of organelle assembly [GO:1902116]; negatively regulates cellulosome assembly [GO:0044575] Also known as: down regulation of cellulosome assembly, down-regulation of cellulosome assembly, downregulation of cellulosome assembly, inhibition of cellulosome assembly